{
  "gene_symbol": "MFGE8",
  "term_id": "GO:0001786",
  "gene": "UniProtKB:Q08431",
  "term_label": "phosphatidylserine binding",
  "gene_name": "Lactadherin"
}